{
  "term_id": "GO:0005739",
  "gene_name": "Methionyl-tRNA formyltransferase, mitochondrial",
  "gene_symbol": "MTFMT",
  "gene": "UniProtKB:Q96DP5",
  "term_label": "mitochondrion"
}